JUN kinase phosphatase activity [GO:0008579] (molecular function) Relationships: is a type of protein tyrosine/serine/threonine phosphatase activity [GO:0008138] Definition: Catalysis of the reaction: JUN kinase serine/threonine/tyrosine phosphate + H2O = JUN kinase serine/threonine/tyrosine + phosphate. Sources: GOC:mah